response to electrical stimulus [GO:0051602] (biological process) Definition: Any process that results in a change in state or activity of a cell or an organism (in terms of movement, secretion, enzyme production, gene expression, etc.) as a result of an electrical stimulus. Sources: GOC:ai Also known as: response to electricity Relationships: is_a GO:0009628 Subtypes: response to electrical stimulus involved in regulation of muscle adaptation [GO:0014878], detection of electrical stimulus [GO:0050981], cellular response to electrical stimulus [GO:0071257], response to immobilization stress combined with electrical stimulus [GO:1990781]